{
  "term_label": "engulfment of apoptotic cell",
  "gene": "UniProtKB:Q5GH72",
  "term_id": "GO:0043652",
  "gene_name": "XK-related protein 7",
  "gene_symbol": "XKR7"
}